{
  "term_label": "plasma membrane",
  "gene_name": "Dedicator of cytokinesis protein 4",
  "gene_symbol": "DOCK4",
  "term_id": "GO:0005886",
  "gene": "UniProtKB:Q8N1I0"
}